{
  "gene_name": "Fibrillin-3",
  "term_label": "extracellular region",
  "term_id": "GO:0005576",
  "gene_symbol": "FBN3",
  "gene": "UniProtKB:Q75N90"
}